{
  "gene": "UniProtKB:Q5MJ70",
  "gene_symbol": "SPDYA",
  "gene_name": "Speedy protein A",
  "term_label": "positive regulation of cell population proliferation",
  "term_id": "GO:0008284"
}